{
  "gene_name": "Ankyrin repeat and SOCS box protein 16",
  "gene": "UniProtKB:Q96NS5",
  "term_label": "Unknown cellular component",
  "gene_symbol": "ASB16",
  "term_id": "UNKNOWN:0003"
}